regulation of bundle of His cell action potential [GO:0098905] (biological process) Also known as: regulation of bundle of His cardiac muscle cell action potential Sources: GOC:BHF, GOC:mtg_cardiac_conduct_nov11 Relationships: is a type of regulation of cardiac muscle cell action potential [GO:0098901]; regulates bundle of His cell action potential [GO:0086043] Definition: Any process that modulates the frequency, rate or extent of action potential creation, propagation or termination in a cardiac muscle cell of the bundle of His. This typically occurs via modulation of the activity or expression of voltage-gated ion channels.